exosporium [GO:0043592] (cellular component) Relationships: is a type of cellular anatomical structure [GO:0110165]; is part of endospore external encapsulating structure [GO:0043591] Definition: The outermost layer of a bacterial endospore, which is loosely attached and located outside of the endospore coat. It is generally composed of protein, carbohydrate, and perhaps lipid. Sources: GOC:mlg Also known as: epispore, exospore, perispore